{
  "gene_name": "NXPE family member 4",
  "gene_symbol": "NXPE4",
  "gene": "UniProtKB:Q6UWF7",
  "term_label": "Unknown biological process",
  "term_id": "UNKNOWN:0002"
}